{
  "term_id": "GO:0030154",
  "term_label": "cell differentiation",
  "gene_symbol": "FOXQ1",
  "gene": "UniProtKB:Q9C009",
  "gene_name": "Forkhead box protein Q1"
}